central tolerance induction [GO:0002508] (biological process) Sources: GOC:jal, GO_REF:0000022, ISBN:0781735149 Relationships: is a type of tolerance induction [GO:0002507] Definition: Tolerance induction in the central lymphoid organs: the thymus and bone marrow. Subtypes: central tolerance induction to nonself antigen [GO:0002463], central tolerance induction to self antigen [GO:0002509], central B cell tolerance induction [GO:0002510], GO:0002512 Regulation: regulated by regulation of central tolerance induction [GO:0002646]; negatively regulated by negative regulation of central tolerance induction [GO:0002647]; positively regulated by GO:0002648